{
  "term_label": "adenylate cyclase-modulating G protein-coupled receptor signaling pathway",
  "gene": "UniProtKB:P63096",
  "gene_name": "Guanine nucleotide-binding protein G(i) subunit alpha-1",
  "term_id": "GO:0007188",
  "gene_symbol": "GNAI1"
}